{
  "gene_name": "Coiled-coil domain-containing protein 182",
  "gene_symbol": "CCDC182",
  "term_id": "UNKNOWN:0001",
  "term_label": "Unknown molecular function",
  "gene": "UniProtKB:A6NF36"
}